{
  "gene_name": "Peroxisomal ATPase PEX1",
  "term_label": "peroxisomal membrane",
  "gene": "UniProtKB:O43933",
  "gene_symbol": "PEX1",
  "term_id": "GO:0005778"
}